regulation of forward locomotion [GO:0043059] (biological process) Sources: GOC:go_curators Subtypes: negative regulation of forward locomotion [GO:1905849], positive regulation of forward locomotion [GO:1905850] Relationships: is a type of GO:0040012; regulates forward locomotion [GO:0043056] Definition: Any process that modulates the speed, mechanical force, or rhythm of the anterior movement of an organism.